{
  "gene": "UniProtKB:P12259",
  "term_label": "Unknown molecular function",
  "gene_name": "Coagulation factor V",
  "term_id": "UNKNOWN:0001",
  "gene_symbol": "F5"
}